{
  "gene_symbol": "RHOV",
  "term_id": "GO:0007015",
  "gene_name": "Rho-related GTP-binding protein RhoV",
  "gene": "UniProtKB:Q96L33",
  "term_label": "actin filament organization"
}